{
  "gene_symbol": "RAB5A",
  "gene": "UniProtKB:P20339",
  "term_id": "GO:0048169",
  "term_label": "regulation of long-term neuronal synaptic plasticity",
  "gene_name": "Ras-related protein Rab-5A"
}